{
  "gene": "UniProtKB:A0A0G2JLJ8",
  "gene_symbol": "IGHD5OR15-5B",
  "gene_name": "Immunoglobulin heavy diversity 5_OR15-5A (non-functional) (Fragment)",
  "term_label": "Unknown biological process",
  "term_id": "UNKNOWN:0002"
}